arabinotriose transport [GO:2001092] (biological process) Sources: GOC:mengo_curators Relationships: is a type of GO:2001088 Definition: The directed movement of an arabinotrioseacetate into, out of or within a cell, or between cells, by means of some agent such as a transporter or pore.